{
  "gene_name": "Transmembrane protein CCDC163",
  "gene": "UniProtKB:A0A0D9SF12",
  "term_id": "UNKNOWN:0001",
  "gene_symbol": "CCDC163",
  "term_label": "Unknown molecular function"
}